{
  "term_id": "GO:0042391",
  "gene_name": "Popeye domain-containing protein 2",
  "term_label": "regulation of membrane potential",
  "gene": "UniProtKB:Q9HBU9",
  "gene_symbol": "POPDC2"
}